{
  "gene_symbol": "TAC4",
  "gene_name": "Tachykinin-4",
  "gene": "UniProtKB:Q86UU9",
  "term_label": "extracellular space",
  "term_id": "GO:0005615"
}